{
  "term_label": "Unknown biological process",
  "gene": "UniProtKB:O14727",
  "gene_name": "Apoptotic protease-activating factor 1",
  "term_id": "UNKNOWN:0002",
  "gene_symbol": "APAF1"
}